{
  "gene_symbol": "NDEL1",
  "term_label": "chromosome localization",
  "term_id": "GO:0050000",
  "gene": "UniProtKB:Q9GZM8",
  "gene_name": "Nuclear distribution protein nudE-like 1"
}